cellular response to insulin stimulus [GO:0032869] (biological process) Definition: Any process that results in a change in state or activity of a cell (in terms of movement, secretion, enzyme production, gene expression, etc.) as a result of an insulin stimulus. Insulin is a polypeptide hormone produced by the islets of Langerhans of the pancreas in mammals, and by the homologous organs of other organisms. Sources: GOC:mah, ISBN:0198506732 Regulation: regulated by regulation of cellular response to insulin stimulus [GO:1900076]; negatively regulated by negative regulation of cellular response to insulin stimulus [GO:1900077]; positively regulated by positive regulation of cellular response to insulin stimulus [GO:1900078] Relationships: is a type of response to insulin [GO:0032868]; is a type of GO:0071375